epithelial tube morphogenesis [GO:0060562] (biological process) Sources: GOC:dph Relationships: is a type of morphogenesis of an epithelium [GO:0002009]; is a type of tube morphogenesis [GO:0035239] Definition: The process in which the anatomical structures of a tube are generated and organized from an epithelium. Epithelial tubes transport gases, liquids and cells from one site to another and form the basic structure of many organs and tissues, with tube shape and organization varying from the single-celled excretory organ in Caenorhabditis elegans to the branching trees of the mammalian kidney and insect tracheal system. Subtypes: embryonic heart tube morphogenesis [GO:0003143], mammary gland duct morphogenesis [GO:0060603], GO:0060652, GO:0061154, renal tubule morphogenesis [GO:0061333], otic vesicle morphogenesis [GO:0071600], metanephric tubule morphogenesis [GO:0072173], nephric duct morphogenesis [GO:0072178]